glycerolipid catabolic process [GO:0046503] (biological process) Also known as: glycerolipid breakdown, glycerolipid catabolism, glycerolipid degradation Sources: GOC:ai Definition: The chemical reactions and pathways resulting in the breakdown of glycerolipids, any lipid with a glycerol backbone. Relationships: is a type of GO:0016042; is a type of glycerolipid metabolic process [GO:0046486] Subtypes: acylglycerol catabolic process [GO:0046464], GO:0046475